{
  "term_id": "GO:0005634",
  "gene_name": "Histone H3.1t",
  "gene_symbol": "H3-4",
  "gene": "UniProtKB:Q16695",
  "term_label": "nucleus"
}